negative regulation of protein catabolic process in the vacuole [GO:1904351] (biological process) Subtypes: negative regulation of lysosomal protein catabolic process [GO:1905166] Also known as: down regulation of protein catabolic process in the vacuole, down-regulation of protein catabolic process in the vacuole, downregulation of protein catabolic process in the vacuole, inhibition of protein catabolic process in the vacuole, down regulation of vacuolar protein breakdown, down regulation of vacuolar protein catabolic process, down regulation of vacuolar protein catabolism, down regulation of vacuolar protein degradation, down-regulation of vacuolar protein breakdown, down-regulation of vacuolar protein catabolic process, down-regulation of vacuolar protein catabolism, down-regulation of vacuolar protein degradation, downregulation of vacuolar protein breakdown, downregulation of vacuolar protein catabolic process, downregulation of vacuolar protein catabolism, downregulation of vacuolar protein degradation, inhibition of vacuolar protein breakdown, inhibition of vacuolar protein catabolic process, inhibition of vacuolar protein catabolism, inhibition of vacuolar protein degradation, negative regulation of vacuolar protein breakdown, negative regulation of vacuolar protein catabolic process, negative regulation of vacuolar protein catabolism, negative regulation of vacuolar protein degradation Relationships: is a type of negative regulation of protein catabolic process [GO:0042177]; is a type of regulation of protein catabolic process in the vacuole [GO:1904350]; negatively regulates protein catabolic process in the vacuole [GO:0007039] Definition: Any process that stops, prevents or reduces the frequency, rate or extent of protein catabolic process in the vacuole. References: PMID:25635054 Sources: GOC:BHF, GOC:TermGenie, GOC:rl, GO_REF:0000058